{
  "term_id": "GO:0050660",
  "gene_name": "Long-chain specific acyl-CoA dehydrogenase, mitochondrial",
  "term_label": "flavin adenine dinucleotide binding",
  "gene": "UniProtKB:P28330",
  "gene_symbol": "ACADL"
}